symbiont-mediated perturbation of host actin cytoskeleton [GO:0141027] (biological process) Also known as: perturbation by symbiont of host actin cytoskeleton, disruption by symbiont of actin cytoskeleton, modification by symbiont of host actin cytoskeleton Subtypes: symbiont-mediated perturbation of host actin cytoskeleton via filamentous actin depolymerization [GO:0141030], symbiont-mediated perturbation of host actin cytoskeleton via actin crosslinking [GO:0141031], symbiont-mediated perturbation of host actin cytoskeleton via actin filament reorganization [GO:0141032], symbiont-mediated perturbation of host actin cytoskeleton via actin polymerization [GO:0141033], symbiont-mediated perturbation of host actin cytoskeleton via inhibition of actin polymerization [GO:0141034] Relationships: is a type of symbiont-mediated perturbation of host cytoskeleton [GO:0052039] Definition: The process in which an organism effects a change that impairs the structure or function of the host actin cytoskeleton. The host is defined as the larger of the organisms involved in a symbiotic interaction. References: PMID:20688909